nicotine catabolic process [GO:0019608] (biological process) Definition: The chemical reactions and pathways resulting in the breakdown of nicotine, (S)(-)-3-(1-methyl-2-pyrrolidinyl)pyridine. Sources: GOC:sm, ISBN:0198547684 Relationships: is a type of GO:0009056; is a type of nicotine metabolic process [GO:0018933] Regulation: positively regulated by positive regulation of nicotine catabolic process [GO:0160160] Also known as: nicotine breakdown, nicotine catabolism, nicotine degradation